{
  "gene_symbol": "ZNF492",
  "term_id": "GO:0000978",
  "term_label": "RNA polymerase II cis-regulatory region sequence-specific DNA binding",
  "gene": "UniProtKB:Q9P255",
  "gene_name": "Zinc finger protein 492"
}